{
  "term_label": "cytoplasm",
  "term_id": "GO:0005737",
  "gene_name": "RILP-like protein 1",
  "gene_symbol": "RILPL1",
  "gene": "UniProtKB:Q5EBL4"
}